{
  "gene": "UniProtKB:Q9P2X3",
  "term_label": "cytoplasm",
  "term_id": "GO:0005737",
  "gene_name": "Protein IMPACT",
  "gene_symbol": "IMPACT"
}